ammonia ligase activity [GO:0016211] (molecular function) Relationships: is a type of GO:0016880 Definition: Catalysis of the ligation of ammonia (NH3) to another substance via a carbon-nitrogen bond with concomitant breakage of a diphosphate linkage, usually in a nucleoside triphosphate. Subtypes: aspartate-ammonia ligase activity [GO:0004071], GO:0004356 Sources: GOC:jl